{
  "term_id": "GO:0006897",
  "gene_name": "Unconventional myosin-Ih",
  "gene_symbol": "MYO1H",
  "term_label": "endocytosis",
  "gene": "UniProtKB:Q8N1T3"
}